{
  "term_label": "heterophilic cell-cell adhesion",
  "gene_name": "Carcinoembryonic antigen-related cell adhesion molecule 6",
  "term_id": "GO:0007157",
  "gene": "UniProtKB:P40199",
  "gene_symbol": "CEACAM6"
}